{
  "gene": "UniProtKB:Q9NPA8",
  "term_id": "GO:0000124",
  "term_label": "SAGA complex",
  "gene_name": "Transcription and mRNA export factor ENY2",
  "gene_symbol": "ENY2"
}